{
  "term_id": "UNKNOWN:0001",
  "gene_symbol": "BRAT1",
  "gene_name": "BRCA1-associated ATM activator 1",
  "term_label": "Unknown molecular function",
  "gene": "UniProtKB:Q6PJG6"
}